{
  "gene": "UniProtKB:Q9NS25",
  "gene_name": "Sperm protein associated with the nucleus on the X chromosome B1",
  "term_id": "UNKNOWN:0003",
  "term_label": "Unknown cellular component",
  "gene_symbol": "SPANXB1"
}